{
  "term_id": "GO:0008543",
  "gene_name": "Fibroblast growth factor receptor 1",
  "term_label": "fibroblast growth factor receptor signaling pathway",
  "gene": "UniProtKB:P11362",
  "gene_symbol": "FGFR1"
}